negative regulation of antimicrobial peptide secretion [GO:0002795] (biological process) Subtypes: negative regulation of antibacterial peptide secretion [GO:0002798], negative regulation of antifungal peptide secretion [GO:0002801] Relationships: is a type of GO:0002785; is a type of negative regulation of peptide secretion [GO:0002792]; is_a regulation of antimicrobial peptide secretion [GO:0002794]; negatively regulates antimicrobial peptide secretion [GO:0002776] Definition: Any process that stops, prevents, or reduces the frequency, rate, or extent of antimicrobial peptide secretion. Sources: GOC:add Also known as: down regulation of antimicrobial peptide secretion, down-regulation of antimicrobial peptide secretion, downregulation of antimicrobial peptide secretion, inhibition of antimicrobial peptide secretion